vasopressin receptor binding [GO:0031893] (MF) Also known as: vasopressin receptor ligand Definition: Binding to a vasopressin receptor. Sources: GOC:mah, GOC:nln Relationships: is a type of G protein-coupled receptor binding [GO:0001664] Subtypes: V1A vasopressin receptor binding [GO:0031894], V1B vasopressin receptor binding [GO:0031895], GO:0031896